{
  "term_label": "calcium-dependent protein binding",
  "term_id": "GO:0048306",
  "gene_symbol": "SNTN",
  "gene_name": "Sentan",
  "gene": "UniProtKB:A6NMZ2"
}